{
  "term_id": "UNKNOWN:0001",
  "gene_name": "Heat shock factor 2-binding protein",
  "gene_symbol": "HSF2BP",
  "term_label": "Unknown molecular function",
  "gene": "UniProtKB:O75031"
}